{
  "term_label": "Unknown biological process",
  "gene": "UniProtKB:P52434",
  "term_id": "UNKNOWN:0002",
  "gene_symbol": "POLR2H",
  "gene_name": "DNA-directed RNA polymerases I, II, and III subunit RPABC3"
}